tryptophan hydroxylase activator activity [GO:0016483] (molecular function) Definition: Increases the activity of the enzyme tryptophase hydroxylase. Relationships: is a type of enzyme activator activity [GO:0008047]; positively regulates tryptophan 5-monooxygenase activity [GO:0004510] Sources: GOC:ai